{
  "gene_symbol": "ACTN2",
  "term_id": "GO:0030864",
  "term_label": "cortical actin cytoskeleton",
  "gene_name": "Alpha-actinin-2",
  "gene": "UniProtKB:P35609"
}